{
  "term_label": "immune response",
  "gene": "UniProtKB:P17693",
  "term_id": "GO:0006955",
  "gene_symbol": "HLA-G",
  "gene_name": "HLA class I histocompatibility antigen, alpha chain G"
}